{
  "term_label": "microtubule cytoskeleton",
  "gene_symbol": "RASSF1",
  "gene": "UniProtKB:Q9NS23",
  "gene_name": "Ras association domain-containing protein 1",
  "term_id": "GO:0015630"
}